{
  "gene": "UniProtKB:P0CG33",
  "gene_symbol": "GOLGA6D",
  "gene_name": "Golgin subfamily A member 6D",
  "term_label": "Golgi cisterna membrane",
  "term_id": "GO:0032580"
}